{
  "term_id": "GO:0000045",
  "term_label": "autophagosome assembly",
  "gene_name": "Activating molecule in BECN1-regulated autophagy protein 1",
  "gene_symbol": "AMBRA1",
  "gene": "UniProtKB:Q9C0C7"
}